catalytic step 1 spliceosome [GO:0071012] (CC) References: PMID:18322460, PMID:19239890 Sources: GOC:ab, GOC:krc, GOC:mah Relationships: is a type of spliceosomal complex [GO:0005681]; is a type of catalytic complex [GO:1902494]; has part Prp19 complex [GO:0000974]; has part U5 snRNP [GO:0005682] Subtypes: GO:0071006, GO:0071017 Definition: A spliceosomal complex that is formed by the displacement of the two snRNPs from the precatalytic spliceosome; three snRNPs including U5 remain associated with the mRNA. This complex, sometimes called the activated spliceosome, is the catalytically active form of the spliceosome, and includes many proteins in addition to those found in the associated snRNPs. Also known as: activated spliceosome, mammalian spliceosomal complex B*, mammalian spliceosomal complex B2, yeast spliceosomal complex A1